{
  "gene_symbol": "MSANTD4",
  "term_label": "Unknown cellular component",
  "term_id": "UNKNOWN:0003",
  "gene": "UniProtKB:Q8NCY6",
  "gene_name": "Myb_SANT-like DNA-binding domain-containing protein 4"
}